{
  "gene": "UniProtKB:P29459",
  "term_label": "cytokine activity",
  "gene_symbol": "IL12A",
  "term_id": "GO:0005125",
  "gene_name": "Interleukin-12 subunit alpha"
}